{
  "term_label": "plasma membrane",
  "gene_symbol": "KIR2DL3",
  "gene": "UniProtKB:P43628",
  "term_id": "GO:0005886",
  "gene_name": "Killer cell immunoglobulin-like receptor 2DL3"
}